Z-phenylacetaldoxime catabolic process [GO:0046308] (BP) Relationships: is a type of catabolic process [GO:0009056]; is a type of GO:0019330 Definition: The chemical reactions and pathways resulting in the breakdown of Z-phenylacetaldoxime, a member of the glucosinolate group of compounds. Sources: GOC:ai Also known as: Z-phenylacetaldoxime breakdown, Z-phenylacetaldoxime catabolism, Z-phenylacetaldoxime degradation